meiotic telophase I [GO:0007134] (biological process) Relationships: is a type of telophase [GO:0051326]; is a type of meiosis I cell cycle phase [GO:0098764] Note: Note that this term should not be used for direct annotation. If you are trying to make an annotation to x phase, it is likely that the correct annotation is 'regulation of x/y phase transition' or to a process which occurs during the reported phase (i.e mitotic DNA replication for mitotic S-phase). To capture the phase when a specific location or process is observed, the phase term can be used in an annotation extension (PMID:24885854) applied to a cellular component term (with the relation exists_during) or a biological process term (with the relation happens_during). Definition: The cell cycle phase which follows anaphase I of meiosis and during which the chromosomes arrive at the poles of the cell and the division of the cytoplasm starts. Sources: GOC:mtg_cell_cycle